{
  "gene_symbol": "CSPG4",
  "gene_name": "Chondroitin sulfate proteoglycan 4",
  "term_id": "GO:0005886",
  "gene": "UniProtKB:Q6UVK1",
  "term_label": "plasma membrane"
}